{
  "gene": "UniProtKB:Q9H6B4",
  "term_label": "Unknown biological process",
  "term_id": "UNKNOWN:0002",
  "gene_symbol": "CLMP",
  "gene_name": "CXADR-like membrane protein"
}